response to platinum ion [GO:0070541] (biological process) Relationships: is_a GO:0010038 Definition: Any process that results in a change in state or activity of a cell or an organism (in terms of movement, secretion, enzyme production, gene expression, etc.) as a result of a platinum stimulus. Sources: GOC:sl Also known as: response to platinum Subtypes: cellular response to platinum ion [GO:0071290]